[tyrosine 3-monooxygenase] kinase activity [GO:0050369] (molecular function) Definition: Catalysis of the reaction: ATP + L-seryl-[tyrosine-3-monooxygenase] = ADP + H+ + O-phospho-L-seryl-[tyrosine-3-monooxygenase]. Relationships: is a type of protein serine/threonine kinase activity [GO:0004674] Also known as: tyrosine 3-monooxygenase kinase activity, ATP:tyrosine-3-monoxygenase phosphotransferase activity, STK4, pheochromocytoma tyrosine hydroxylase-associated kinase activity, tyrosine 3-monooxygenase kinase (phosphorylating) activity Sources: EC:2.7.11.6